{
  "gene_name": "RING-type E3 ubiquitin-protein ligase PPIL2",
  "term_label": "Unknown biological process",
  "gene": "UniProtKB:Q13356",
  "gene_symbol": "PPIL2",
  "term_id": "UNKNOWN:0002"
}